cellular response to carbon dioxide [GO:0071244] (BP) Sources: GOC:mah Definition: Any process that results in a change in state or activity of a cell (in terms of movement, secretion, enzyme production, gene expression, etc.) as a result of a carbon dioxide (CO2) stimulus. Relationships: is a type of GO:0010037; is a type of cellular response to oxygen-containing compound [GO:1901701]